{
  "gene": "UniProtKB:O15481",
  "term_label": "Unknown molecular function",
  "gene_name": "Melanoma-associated antigen B4",
  "gene_symbol": "MAGEB4",
  "term_id": "UNKNOWN:0001"
}